oligosaccharyltransferase complex B [GO:0160227] (cellular component) Definition: An oligosaccharyltransferase complex that contains STT3B as the catalytic subunit. Relationships: is a type of oligosaccharyltransferase complex [GO:0008250] References: PMID:31831667, PMID:39509507 Also known as: OST-B